{
  "gene": "UniProtKB:O95522",
  "term_id": "GO:0031462",
  "gene_symbol": "PRAMEF12",
  "term_label": "Cul2-RING ubiquitin ligase complex",
  "gene_name": "PRAME family member 12"
}